microtubule-dependent intracellular transport of viral material towards cell periphery [GO:0039701] (biological process) Definition: The directed movement of the viral genome or a viral particle towards the cell periphery using host microtubules. Mostly used by viruses that replicate their genome near or in the nucleus to allows newly assembled viral progeny to reach the plasma membrane. Relationships: is a type of microtubule-dependent intracellular transport of viral material [GO:0075519] Sources: UniProtKB-KW:KW-1189, VZ:1816